{
  "gene": "UniProtKB:Q15761",
  "gene_name": "Neuropeptide Y receptor type 5",
  "gene_symbol": "NPY5R",
  "term_id": "GO:0007218",
  "term_label": "neuropeptide signaling pathway"
}